{
  "term_id": "UNKNOWN:0002",
  "gene": "UniProtKB:Q63HM2",
  "gene_name": "Pecanex-like protein 4",
  "term_label": "Unknown biological process",
  "gene_symbol": "PCNX4"
}